{
  "gene_name": "Aquaporin-7",
  "term_label": "glycerol transmembrane transport",
  "term_id": "GO:0015793",
  "gene": "UniProtKB:O14520",
  "gene_symbol": "AQP7"
}